{
  "gene_symbol": "PDE2A",
  "term_label": "mitochondrial outer membrane",
  "term_id": "GO:0005741",
  "gene_name": "cGMP-dependent 3',5'-cyclic phosphodiesterase",
  "gene": "UniProtKB:O00408"
}